{
  "gene": "UniProtKB:Q9NW68",
  "term_id": "GO:0005737",
  "gene_symbol": "BSDC1",
  "term_label": "cytoplasm",
  "gene_name": "BSD domain-containing protein 1"
}